{
  "term_label": "regulation of viral entry into host cell",
  "gene_name": "Tripartite motif-containing protein 5",
  "gene": "UniProtKB:Q9C035",
  "term_id": "GO:0046596",
  "gene_symbol": "TRIM5"
}